{
  "gene_name": "Protein S100-A12",
  "gene": "UniProtKB:P80511",
  "term_id": "GO:0005509",
  "term_label": "calcium ion binding",
  "gene_symbol": "S100A12"
}